auxin binding [GO:0010011] (molecular function) Also known as: auxin receptor Relationships: is a type of hormone binding [GO:0042562] Definition: Binding to auxin, a plant hormone that regulates aspects of plant growth. Sources: GOC:sm